{
  "gene": "UniProtKB:Q9BV81",
  "gene_name": "ER membrane protein complex subunit 6",
  "term_id": "GO:0072546",
  "gene_symbol": "EMC6",
  "term_label": "EMC complex"
}